{
  "term_label": "endoplasmic reticulum membrane",
  "gene_symbol": "VTI1A",
  "gene": "UniProtKB:Q96AJ9",
  "term_id": "GO:0005789",
  "gene_name": "Vesicle transport through interaction with t-SNAREs homolog 1A"
}